{
  "gene_symbol": "BSPH1",
  "term_label": "cell surface",
  "gene_name": "Binder of sperm protein homolog 1",
  "term_id": "GO:0009986",
  "gene": "UniProtKB:Q075Z2"
}